{
  "term_id": "GO:0015629",
  "gene": "UniProtKB:Q8TDY3",
  "gene_name": "Actin-related protein T2",
  "gene_symbol": "ACTRT2",
  "term_label": "actin cytoskeleton"
}